{
  "gene": "UniProtKB:O60347",
  "term_label": "regulation of autophagosome assembly",
  "gene_symbol": "TBC1D12",
  "term_id": "GO:2000785",
  "gene_name": "TBC1 domain family member 12"
}